SWI/SNF complex [GO:0016514] (cellular component) Also known as: SWI-SNF complex Definition: A SWI/SNF-type complex that contains 8 to 14 proteins, including both conserved (core) and nonconserved components; contains the ATPase product of the yeast SNF2 or mammalian SMARCA4/BAF190A/BRG1 gene, or an ortholog thereof. Relationships: is_a SWI/SNF superfamily-type complex [GO:0070603] References: PMID:12672490 Sources: GOC:bhm